{
  "gene": "UniProtKB:P02708",
  "gene_symbol": "CHRNA1",
  "term_id": "GO:0022848",
  "gene_name": "Acetylcholine receptor subunit alpha",
  "term_label": "acetylcholine-gated monoatomic cation-selective channel activity"
}